{
  "term_label": "G protein-coupled receptor signaling pathway",
  "gene": "UniProtKB:Q8NGL0",
  "gene_symbol": "OR5L2",
  "gene_name": "Olfactory receptor 5L2",
  "term_id": "GO:0007186"
}